{
  "term_label": "galactosylceramide catabolic process",
  "gene_symbol": "GALC",
  "gene": "UniProtKB:P54803",
  "term_id": "GO:0006683",
  "gene_name": "Galactocerebrosidase"
}